{
  "gene_name": "Leucine-rich repeat-containing protein 26",
  "gene_symbol": "LRRC26",
  "term_id": "UNKNOWN:0002",
  "term_label": "Unknown biological process",
  "gene": "UniProtKB:Q2I0M4"
}